hyphal cell wall [GO:0030446] (cellular component) Definition: The cell wall surrounding a fungal hypha. Sources: GOC:mah Note: See also the Fungal Anatomy Ontology term 'hypha ; FAO:0001001'. Relationships: is a type of GO:0009277